{
  "gene": "UniProtKB:Q6ZSR3",
  "term_label": "Unknown molecular function",
  "gene_name": "Putative uncharacterized protein FLJ45275, mitochondrial",
  "term_id": "UNKNOWN:0001",
  "gene_symbol": "Q6ZSR3"
}